{
  "gene": "UniProtKB:P54707",
  "term_label": "plasma membrane",
  "term_id": "GO:0005886",
  "gene_name": "Potassium-transporting ATPase alpha chain 2",
  "gene_symbol": "ATP12A"
}